{
  "gene_name": "Cell adhesion molecule DSCAM",
  "term_id": "GO:0043025",
  "gene_symbol": "DSCAM",
  "term_label": "neuronal cell body",
  "gene": "UniProtKB:O60469"
}